{
  "term_label": "Unknown molecular function",
  "gene": "UniProtKB:Q5VXT5",
  "term_id": "UNKNOWN:0001",
  "gene_symbol": "SYPL2",
  "gene_name": "Synaptophysin-like protein 2"
}